negative regulation of protein localization to ciliary membrane [GO:1903568] (biological process) Definition: Any process that stops, prevents or reduces the frequency, rate or extent of protein localization to ciliary membrane. Also known as: down regulation of protein localisation in ciliary membrane, down regulation of protein localisation to ciliary membrane, down regulation of protein localization in ciliary membrane, down regulation of protein localization to ciliary membrane, down-regulation of protein localisation in ciliary membrane, down-regulation of protein localisation to ciliary membrane, down-regulation of protein localization in ciliary membrane, down-regulation of protein localization to ciliary membrane, downregulation of protein localisation in ciliary membrane, downregulation of protein localisation to ciliary membrane, downregulation of protein localization in ciliary membrane, downregulation of protein localization to ciliary membrane, negative regulation of protein localisation in ciliary membrane, negative regulation of protein localisation to ciliary membrane, negative regulation of protein localization in ciliary membrane, inhibition of protein localisation in ciliary membrane, inhibition of protein localisation to ciliary membrane, inhibition of protein localization in ciliary membrane, inhibition of protein localization to ciliary membrane References: PMID:22072986 Sources: GOC:TermGenie, GOC:cilia, GOC:krc, GO_REF:0000058 Relationships: is a type of GO:1903565; is a type of regulation of protein localization to ciliary membrane [GO:1903567]; is a type of negative regulation of protein localization to cell periphery [GO:1904376]; is a type of GO:1905476; RO_0002212 protein localization to ciliary membrane [GO:1903441]